octanol dehydrogenase (NAD+) activity [GO:0004552] (molecular function) Also known as: octanol dehydrogenase activity, 1-octanol dehydrogenase activity, octanol:NAD+ oxidoreductase activity Definition: Catalysis of the reaction: 1-octanol + NAD+ = 1-octanal + H+ + NADH. Relationships: is a type of alcohol dehydrogenase (NAD+) activity [GO:0004022] Sources: EC:1.1.1.73, RHEA:24620